endosperm development [GO:0009960] (biological process) Regulation: negatively regulated by negative regulation of endosperm development [GO:1904095]; regulated by regulation of endosperm development [GO:2000014] Sources: GOC:sm Definition: The process whose specific outcome is the progression of the endosperm over time, from its formation to the mature structure. The endosperm is formed during fertilization and provides nutrients to the developing embryo. Relationships: is a type of GO:0003006; is a type of tissue development [GO:0009888]; is part of seed development [GO:0048316]